{
  "term_label": "immune response",
  "gene_symbol": "IGLV1-50",
  "gene_name": "Probable non-functional immunoglobulin lambda variable 1-50",
  "gene": "UniProtKB:A0A075B6I6",
  "term_id": "GO:0006955"
}